{
  "gene_symbol": "TSC2",
  "term_id": "GO:0046627",
  "gene": "UniProtKB:P49815",
  "term_label": "negative regulation of insulin receptor signaling pathway",
  "gene_name": "Tuberin"
}